{
  "gene": "UniProtKB:Q9UPT8",
  "gene_symbol": "ZC3H4",
  "gene_name": "Zinc finger CCCH domain-containing protein 4",
  "term_label": "DNA-binding transcription repressor activity, RNA polymerase II-specific",
  "term_id": "GO:0001227"
}